{
  "term_label": "nucleus",
  "gene_symbol": "ZNF696",
  "gene": "UniProtKB:Q9H7X3",
  "term_id": "GO:0005634",
  "gene_name": "Zinc finger protein 696"
}